{
  "term_label": "vesicle fusion",
  "term_id": "GO:0006906",
  "gene": "UniProtKB:Q15836",
  "gene_symbol": "VAMP3",
  "gene_name": "Vesicle-associated membrane protein 3"
}